{
  "term_id": "GO:0009267",
  "gene_name": "Serine_threonine-protein kinase PAK 6",
  "gene": "UniProtKB:Q9NQU5",
  "term_label": "cellular response to starvation",
  "gene_symbol": "PAK6"
}